{
  "term_label": "Unknown molecular function",
  "gene": "UniProtKB:O43676",
  "gene_name": "NADH dehydrogenase [ubiquinone] 1 beta subcomplex subunit 3",
  "term_id": "UNKNOWN:0001",
  "gene_symbol": "NDUFB3"
}